{
  "gene_name": "Omega-amidase NIT2",
  "gene_symbol": "NIT2",
  "gene": "UniProtKB:Q9NQR4",
  "term_id": "GO:0006107",
  "term_label": "oxaloacetate metabolic process"
}